{
  "gene_symbol": "CTAG2",
  "gene": "UniProtKB:O75638",
  "term_label": "Unknown molecular function",
  "term_id": "UNKNOWN:0001",
  "gene_name": "Cancer_testis antigen 2"
}